embryonic organ morphogenesis [GO:0048562] (biological process) Relationships: is a type of animal organ morphogenesis [GO:0009887]; is a type of embryonic morphogenesis [GO:0048598]; is part of GO:0048568 Subtypes: GO:0030538, ear morphogenesis [GO:0042471], embryonic eye morphogenesis [GO:0048048], embryonic digestive tract morphogenesis [GO:0048557], notochord morphogenesis [GO:0048570], embryonic skeletal system morphogenesis [GO:0048704], otic vesicle morphogenesis [GO:0071600] Definition: Morphogenesis, during the embryonic phase, of a tissue or tissues that work together to perform a specific function or functions. Morphogenesis is the process in which anatomical structures are generated and organized. Organs are commonly observed as visibly distinct structures, but may also exist as loosely associated clusters of cells that work together to perform a specific function or functions. Sources: GOC:jid